{
  "term_label": "regulation of mitotic cytokinesis",
  "gene_symbol": "ANKRD53",
  "gene_name": "Ankyrin repeat domain-containing protein 53",
  "gene": "UniProtKB:Q8N9V6",
  "term_id": "GO:1902412"
}